phloem sucrose unloading [GO:0110128] (biological process) Definition: The process of unloading sucrose that is produced in the source tissues, from the sieve tube or companion cell of the phloem into the sink tissues. Relationships: is a type of sucrose transport [GO:0015770]; is a type of phloem unloading [GO:0110127] References: PMID:30018170 Sources: GOC:lr